{
  "gene_name": "Pejvakin",
  "gene": "UniProtKB:Q0ZLH3",
  "term_id": "UNKNOWN:0001",
  "gene_symbol": "PJVK",
  "term_label": "Unknown molecular function"
}